resolution phase response [GO:0106299] (biological process) Relationships: is a type of acute inflammatory response [GO:0002526] Definition: An active host response phase of acute inflammation driven by specialized pro-resolving mediators (SPMs) and signaling pathways, enabling timely tissue regeneration and return of function. Note: Acute inflammatory response(s) are self-limited, resolve on their own and classically divide into initiation and resolution phases. SPMs are a superfamily of proresolving mediators that include resolvins (Rvs), protectins (PDs), maresins (MaRs) and lipoxins (LXs). References: PMID:28087575